{
  "gene_name": "SMAD5 antisense gene protein 1",
  "term_id": "UNKNOWN:0002",
  "term_label": "Unknown biological process",
  "gene_symbol": "SMAD5-AS1",
  "gene": "UniProtKB:Q9Y6J3"
}